{
  "gene_symbol": "DNAAF4",
  "term_id": "GO:0030331",
  "gene": "UniProtKB:Q8WXU2",
  "gene_name": "Dynein axonemal assembly factor 4",
  "term_label": "nuclear estrogen receptor binding"
}